{
  "gene_symbol": "ENTPD5",
  "gene_name": "Nucleoside diphosphate phosphatase ENTPD5",
  "gene": "UniProtKB:O75356",
  "term_id": "UNKNOWN:0002",
  "term_label": "Unknown biological process"
}